{
  "term_label": "catenin complex",
  "term_id": "GO:0016342",
  "gene_name": "Cadherin-15",
  "gene_symbol": "CDH15",
  "gene": "UniProtKB:P55291"
}